{
  "gene_name": "Syntaxin-17",
  "gene": "UniProtKB:P56962",
  "gene_symbol": "STX17",
  "term_label": "exocytosis",
  "term_id": "GO:0006887"
}